{
  "gene_symbol": "RBM15",
  "term_id": "GO:0003729",
  "term_label": "mRNA binding",
  "gene": "UniProtKB:Q96T37",
  "gene_name": "RNA-binding protein 15"
}